{
  "gene": "UniProtKB:P06396",
  "term_label": "cell projection assembly",
  "term_id": "GO:0030031",
  "gene_symbol": "GSN",
  "gene_name": "Gelsolin"
}